divisome complex [GO:1990586] (CC) Subtypes: GO:1990587, GO:1990588 References: PMID:15165235, PMID:21784946 Sources: GOC:bhm Relationships: is a type of protein-containing complex [GO:0032991]; is part of cell septum [GO:0030428] Definition: A protein complex required for prokaryotic cell division (FtsZ-dependent cytokinesis). These complexes are assembled and recruited to the cell septum in a strictly controlled sequence and co-ordinate invagination of the cell membrane, inward growth of the peptidoglycan layer, constriction of the outer membrane and separation of daughter cells.